positive regulation of chromosome passenger complex localization to kinetochore [GO:0140430] (biological process) Relationships: is a type of positive regulation of protein localization to kinetochore [GO:1905342]; positively regulates chromosome passenger complex localization to kinetochore [GO:0072356] References: PMID:20739936 Definition: Any process that activates or increases the frequency, rate or extent of a chromosome passenger complex localization to kinetochore.